{
  "gene_name": "RAC-beta serine_threonine-protein kinase",
  "gene_symbol": "AKT2",
  "term_id": "GO:0035556",
  "gene": "UniProtKB:P31751",
  "term_label": "intracellular signal transduction"
}